{
  "gene_name": "PH-interacting protein",
  "gene_symbol": "PHIP",
  "term_label": "nucleus",
  "term_id": "GO:0005634",
  "gene": "UniProtKB:Q8WWQ0"
}